{
  "gene_symbol": "FHIP2B",
  "gene": "UniProtKB:Q86V87",
  "term_label": "Unknown biological process",
  "gene_name": "FHF complex subunit HOOK-interacting protein 2B",
  "term_id": "UNKNOWN:0002"
}